{
  "term_id": "GO:0005730",
  "term_label": "nucleolus",
  "gene": "UniProtKB:Q9P1T7",
  "gene_symbol": "MDFIC",
  "gene_name": "MyoD family inhibitor domain-containing protein"
}